{
  "gene": "UniProtKB:Q9UII2",
  "gene_symbol": "ATP5IF1",
  "gene_name": "ATPase inhibitor, mitochondrial",
  "term_id": "GO:0006783",
  "term_label": "heme biosynthetic process"
}